{
  "term_id": "GO:0005930",
  "gene": "UniProtKB:Q9H0K4",
  "gene_name": "Radial spoke head protein 6 homolog A",
  "gene_symbol": "RSPH6A",
  "term_label": "axoneme"
}